negative regulation of endothelial cell chemotaxis to vascular endothelial growth factor [GO:1904858] (biological process) Relationships: is a type of negative regulation of cell migration [GO:0030336]; is a type of negative regulation of chemotaxis [GO:0050922]; is a type of negative regulation of cellular response to vascular endothelial growth factor stimulus [GO:1902548]; is a type of GO:1904857; negatively regulates endothelial cell chemotaxis to vascular endothelial growth factor [GO:0090668] References: PMID:21885851 Sources: GOC:BHF, GOC:BHF_miRNA, GOC:TermGenie, GOC:rph, GO_REF:0000058 Also known as: down regulation of endothelial cell chemotaxis to vascular endothelial growth factor, down-regulation of endothelial cell chemotaxis to vascular endothelial growth factor, downregulation of endothelial cell chemotaxis to vascular endothelial growth factor, inhibition of endothelial cell chemotaxis to vascular endothelial growth factor Definition: Any process that stops, prevents or reduces the frequency, rate or extent of endothelial cell chemotaxis to vascular endothelial growth factor.